{
  "gene_name": "Claudin-1",
  "gene_symbol": "CLDN1",
  "gene": "UniProtKB:O95832",
  "term_label": "virus receptor activity",
  "term_id": "GO:0001618"
}